{
  "gene_name": "Kelch-like protein 15",
  "gene": "UniProtKB:Q96M94",
  "gene_symbol": "KLHL15",
  "term_id": "GO:0005634",
  "term_label": "nucleus"
}